{
  "gene": "UniProtKB:H0Y354",
  "gene_name": "Protein FAM72C",
  "gene_symbol": "FAM72C",
  "term_id": "GO:0005829",
  "term_label": "cytosol"
}